{
  "term_id": "GO:0000289",
  "gene_symbol": "ZFP36L1",
  "term_label": "nuclear-transcribed mRNA poly(A) tail shortening",
  "gene_name": "mRNA decay activator protein ZFP36L1",
  "gene": "UniProtKB:Q07352"
}